{
  "term_id": "GO:0070578",
  "term_label": "RISC-loading complex",
  "gene_symbol": "PRKRA",
  "gene_name": "Interferon-inducible double-stranded RNA-dependent protein kinase activator A",
  "gene": "UniProtKB:O75569"
}